{
  "gene_name": "Gamma-aminobutyric acid receptor subunit rho-3",
  "gene": "UniProtKB:A8MPY1",
  "term_id": "GO:0004890",
  "gene_symbol": "GABRR3",
  "term_label": "GABA-A receptor activity"
}